negative regulation of ribosome biogenesis [GO:0090071] (biological process) Sources: GOC:dph, GOC:tb Subtypes: GO:2000201, negative regulation of rRNA processing [GO:2000233] Definition: Any process that decreases the rate, frequency or extent of ribosome biogenesis. Ribosome biogenesis is the cellular process that results in the biosynthesis of constituent macromolecules, assembly, and arrangement of constituent parts of ribosome subunits. Relationships: is a type of negative regulation of cellular process [GO:0048523]; is a type of regulation of ribosome biogenesis [GO:0090069]; negatively regulates ribosome biogenesis [GO:0042254]